{
  "gene_name": "A disintegrin and metalloproteinase with thrombospondin motifs 4",
  "term_id": "GO:0006508",
  "gene_symbol": "ADAMTS4",
  "term_label": "proteolysis",
  "gene": "UniProtKB:O75173"
}